{
  "gene_name": "Ras-related protein Rab-11B",
  "term_label": "recycling endosome",
  "term_id": "GO:0055037",
  "gene": "UniProtKB:Q15907",
  "gene_symbol": "RAB11B"
}